galacturonate catabolic process [GO:0046397] (biological process) Definition: The chemical reactions and pathways resulting in the breakdown of galacturonate, the anion of galacturonic acid. Sources: GOC:ai Subtypes: D-galacturonate catabolic process [GO:0019698] Relationships: is a type of GO:0072329 Also known as: galacturonate breakdown, galacturonate catabolism, galacturonate degradation